cysteine-type endopeptidase activator activity [GO:0140608] (molecular function) Relationships: is a type of endopeptidase activator activity [GO:0061133]; positively regulates GO:0004197 References: PMID:32558991 Definition: Binds to and increases the activity of a cysteine-type endopeptidase. Also known as: caspase activator activator activity